{
  "term_id": "UNKNOWN:0002",
  "gene_name": "Beckwith-Wiedemann syndrome chromosomal region 1 candidate gene B protein",
  "term_label": "Unknown biological process",
  "gene": "UniProtKB:Q8N1D0",
  "gene_symbol": "SLC22A18AS"
}